{
  "gene": "UniProtKB:P10276",
  "term_id": "GO:0000978",
  "gene_symbol": "RARA",
  "term_label": "RNA polymerase II cis-regulatory region sequence-specific DNA binding",
  "gene_name": "Retinoic acid receptor alpha"
}